{
  "gene_name": "Transmembrane protein 100",
  "term_id": "GO:0051930",
  "term_label": "regulation of sensory perception of pain",
  "gene": "UniProtKB:Q9NV29",
  "gene_symbol": "TMEM100"
}